{
  "gene": "UniProtKB:Q8WY54",
  "term_label": "signal transduction",
  "gene_name": "Protein phosphatase 1E",
  "gene_symbol": "PPM1E",
  "term_id": "GO:0007165"
}